{
  "term_label": "detection of chemical stimulus involved in sensory perception of smell",
  "gene_name": "Olfactory receptor 6Q1",
  "gene": "UniProtKB:Q8NGQ2",
  "gene_symbol": "OR6Q1",
  "term_id": "GO:0050911"
}